{
  "gene_name": "GRB2-related adapter protein 2",
  "term_label": "phosphotyrosine residue binding",
  "term_id": "GO:0001784",
  "gene_symbol": "GRAP2",
  "gene": "UniProtKB:O75791"
}